negative regulation of vitamin metabolic process [GO:0046137] (BP) Sources: GOC:ai Relationships: is a type of regulation of vitamin metabolic process [GO:0030656]; is a type of GO:0062014; negatively regulates vitamin metabolic process [GO:0006766] Subtypes: GO:0010957, negative regulation of thiamine diphosphate biosynthetic process [GO:0070617], negative regulation of thiamine biosynthetic process [GO:0070624], negative regulation of retinoic acid biosynthetic process [GO:1900053], negative regulation of L-ascorbic acid biosynthetic process [GO:2000083] Also known as: down regulation of vitamin metabolic process, down-regulation of vitamin metabolic process, downregulation of vitamin metabolic process, negative regulation of vitamin metabolism, inhibition of vitamin metabolic process Definition: Any process that stops, prevents, or reduces the frequency, rate or extent of the chemical reactions and pathways involving a vitamin, one of a number of unrelated organic substances that occur in many foods in small amounts and that are necessary in trace amounts for the normal metabolic functioning of the body.